{
  "gene_symbol": "PTPRD",
  "gene": "UniProtKB:P23468",
  "term_id": "GO:0099560",
  "term_label": "synaptic membrane adhesion",
  "gene_name": "Receptor-type tyrosine-protein phosphatase delta"
}